{
  "gene_symbol": "RTN4IP1",
  "term_label": "mitochondrion",
  "term_id": "GO:0005739",
  "gene": "UniProtKB:Q8WWV3",
  "gene_name": "Reticulon-4-interacting protein 1, mitochondrial"
}